{
  "term_id": "GO:0030154",
  "gene_name": "Matrix remodeling-associated protein 8",
  "term_label": "cell differentiation",
  "gene_symbol": "MXRA8",
  "gene": "UniProtKB:Q9BRK3"
}